leucoplast fission [GO:0043573] (biological process) Sources: GOC:jl Relationships: is a type of plastid fission [GO:0043572] Definition: The creation of two or more leucoplasts by division of one leucoplast. A leucoplast is a colorless plastid involved in the synthesis of monoterpenes.